{
  "gene": "UniProtKB:Q6HA08",
  "term_label": "extracellular space",
  "gene_name": "Astacin-like metalloendopeptidase",
  "term_id": "GO:0005615",
  "gene_symbol": "ASTL"
}